{
  "gene_name": "Saitohin",
  "term_label": "Unknown molecular function",
  "gene": "UniProtKB:Q8IWL8",
  "gene_symbol": "STH",
  "term_id": "UNKNOWN:0001"
}